{
  "gene_name": "Polypyrimidine tract-binding protein 2",
  "term_id": "GO:0003729",
  "gene_symbol": "PTBP2",
  "gene": "UniProtKB:Q9UKA9",
  "term_label": "mRNA binding"
}